lipopolysaccharide transfer activity [GO:0140332] (molecular function) Definition: Removes a lipopolysaccharide (LPS) from the outer leaflet of a donor membrane, transports it through the aqueous phase while protected in a hydrophobic pocket, and brings it to the outer leaflet of an acceptor membrane. Relationships: is a type of lipid transfer activity [GO:0120013]; is part of lipopolysaccharide transport [GO:0015920] References: PMID:24639492 Also known as: intermembrane LPS transporter activity, intermembrane lipopolysaccharide transfer activity, intermembrane lipopolysaccharide transporter activity, lipopolysaccharide carrier activity